guanine deglycation, methylglyoxal removal [GO:0106045] (BP) Relationships: is a type of GO:0009438; is a type of GO:0106044; is a type of cellular detoxification of methylglyoxal [GO:0140041] Definition: The removal of methylglyoxal from a glycated guanine, to form lactate and a deglycated guanine. References: PMID:28596309